emericellamide A biosynthetic process [GO:1900617] (biological process) Definition: The chemical reactions and pathways resulting in the formation of emericellamide A. Regulation: regulated by regulation of emericellamide A biosynthetic process [GO:1900661]; negatively regulated by negative regulation of emericellamide A biosynthetic process [GO:1900662]; positively regulated by positive regulation of emericellamide A biosynthetic process [GO:1900663] Relationships: is a type of emericellamide biosynthetic process [GO:1900557] Also known as: emericellamide A anabolism, emericellamide A biosynthesis, emericellamide A formation, emericellamide A synthesis Sources: GOC:TermGenie, GOC:di